{
  "gene_name": "Ribonuclease SLFN12",
  "term_id": "UNKNOWN:0001",
  "gene": "UniProtKB:Q8IYM2",
  "gene_symbol": "SLFN12",
  "term_label": "Unknown molecular function"
}